{
  "term_id": "GO:0007166",
  "gene_name": "T cell receptor beta variable 7-7",
  "term_label": "cell surface receptor signaling pathway",
  "gene": "UniProtKB:A0A0K0K1E9",
  "gene_symbol": "TRBV7-7"
}